negative regulation of antifungal peptide biosynthetic process [GO:0002811] (biological process) Also known as: down regulation of antifungal peptide biosynthetic process, down-regulation of antifungal peptide biosynthetic process, downregulation of antifungal peptide biosynthetic process, inhibition of antifungal peptide biosynthetic process Sources: GOC:add Relationships: is a type of negative regulation of antifungal peptide production [GO:0002789]; is a type of GO:0002806; is a type of regulation of antifungal peptide biosynthetic process [GO:0002810]; negatively regulates antifungal peptide biosynthetic process [GO:0002783] Definition: Any process that stops, prevents, or reduces the frequency, rate, or extent of antifungal peptide biosynthesis.